IscS-TusA complex [GO:1990329] (cellular component) Definition: A heterotetrameric protein complex involved in the sulfur-relay system required for 2-thiolation of 5-methylaminomethyl-2-thiouridine (mnm5s2U) at tRNA wobble positions. In E. coli it consists of a central IscS dimer with the two TusA protomers bound to one of the IscS units each via persulfide (-SSH) groups. Relationships: is a type of L-cysteine desulfurase complex [GO:1990221] References: PMID:20404999 Sources: GOC:bhm